hemocyte differentiation [GO:0042386] (biological process) Relationships: is a type of immune system process [GO:0002376]; is a type of cell differentiation [GO:0030154] Subtypes: embryonic hemocyte differentiation [GO:0035163], larval lymph gland hemocyte differentiation [GO:0035168], GO:0042387, GO:0042688 Also known as: arthropod blood cell differentiation Regulation: regulated by regulation of hemocyte differentiation [GO:0045610]; negatively regulated by negative regulation of hemocyte differentiation [GO:0045611]; positively regulated by positive regulation of hemocyte differentiation [GO:0045612] References: PMID:9550723 Sources: CL:0000387, GOC:jl, GOC:mtg_sensu Definition: The process in which a relatively unspecialized cell acquires the characteristics of a mature hemocyte. Hemocytes are blood cells associated with a hemocoel (the cavity containing most of the major organs of the arthropod body) which are involved in defense and clotting of hemolymph, but not involved in transport of oxygen.